steroid 11-beta-monooxygenase activity [GO:0004507] (molecular function) Also known as: steroid 11-beta-hydroxylase activity, cytochrome P450 CYP11B1, cytochrome P450 CYP11B2, cytochrome p450 XIB1 activity, oxygenase, steroid 11beta -mono-, steroid 11-beta/18-hydroxylase activity, steroid 11beta-hydroxylase activity, steroid 11beta-monooxygenase activity, steroid 11beta/18-hydroxylase activity, steroid,reduced-adrenal-ferredoxin:oxygen oxidoreductase (11beta-hydroxylating) Sources: EC:1.14.15.4 Definition: Catalysis of the reaction: a steroid + reduced adrenal ferredoxin + O2 = an 11-beta-hydroxysteroid + oxidized adrenal ferredoxin + H2O. Relationships: is a type of GO:0008395; is a type of oxidoreductase activity, acting on paired donors, with incorporation or reduction of molecular oxygen, reduced iron-sulfur protein as one donor, and incorporation of one atom of oxygen [GO:0016713]